{
  "gene": "UniProtKB:Q2TAA5",
  "term_label": "GDP-Man:Man(3)GlcNAc(2)-PP-Dol alpha-1,2-mannosyltransferase activity",
  "gene_name": "GDP-Man:Man(3)GlcNAc(2)-PP-Dol alpha-1,2-mannosyltransferase",
  "gene_symbol": "ALG11",
  "term_id": "GO:0004377"
}